{
  "gene_symbol": "MICU2",
  "term_id": "GO:0005509",
  "gene": "UniProtKB:Q8IYU8",
  "gene_name": "Calcium uptake protein 2, mitochondrial",
  "term_label": "calcium ion binding"
}